ubiquinone metabolic process [GO:0006743] (BP) Sources: GOC:mah Also known as: coenzyme Q metabolic process, coenzyme Q metabolism, ubiquinone metabolism Definition: The chemical reactions and pathways involving ubiquinone, a lipid-soluble electron-transporting coenzyme. Relationships: is a type of quinone metabolic process [GO:1901661] Subtypes: ubiquinone biosynthetic process [GO:0006744], ubiquinone catabolic process [GO:0032322]